{
  "term_label": "microtubule anchoring at centrosome",
  "term_id": "GO:0034454",
  "gene": "UniProtKB:Q8N4C6",
  "gene_symbol": "NIN",
  "gene_name": "Ninein"
}